histone H3K4me1 reader activity [GO:0140109] (molecular function) Relationships: is a type of histone H3 reader activity [GO:0140006] References: PMID:18840606, PMID:29255264 Also known as: H3-K4me1 modified histone binding, H3K4me1 modified histone binding Definition: A histone reader that recognizes a histone H3 monomethylated at lysine 4. Note: Comment: Note that the residue position corresponds to the canonical human H3 histone (UniProtKB:P84243); this residue is conserved across all eukaryotes. Residue 1 is the first residue following removal of the initiating Methionine (Met). Note that each histone is encoded by multiple genes, and sequences may vary across different genes within an organism.